positive regulation of protein localization to endosome [GO:1905668] (BP) References: PMID:22732145 Sources: GOC:PARL, GOC:TermGenie, GOC:bc, GO_REF:0000058 Also known as: positive regulation of protein localisation in endosome, positive regulation of protein localization in endosome, up regulation of protein localisation in endosome, up regulation of protein localization in endosome, up regulation of protein localization to endosome, up-regulation of protein localisation in endosome, up-regulation of protein localization in endosome, up-regulation of protein localization to endosome, upregulation of protein localisation in endosome, upregulation of protein localization in endosome, upregulation of protein localization to endosome, activation of protein localisation in endosome, activation of protein localization in endosome, activation of protein localization to endosome Subtypes: GO:1902966 Relationships: is a type of positive regulation of protein localization [GO:1903829]; is a type of GO:1905666; positively regulates protein localization to endosome [GO:0036010] Definition: Any process that activates or increases the frequency, rate or extent of protein localization to endosome.